{
  "term_id": "UNKNOWN:0001",
  "gene_symbol": "CARTPT",
  "term_label": "Unknown molecular function",
  "gene": "UniProtKB:Q16568",
  "gene_name": "Cocaine- and amphetamine-regulated transcript protein"
}